beta-nitroacrylate reductase activity [GO:0047703] (molecular function) Definition: Catalysis of the reaction: 3-nitropropanoate + NADP+ = 3-nitroacrylate + H+ + NADPH. Sources: EC:1.3.1.16, RHEA:23892 Also known as: b-nitroacrylate reductase activity, 3-nitropropanoate:NADP+ oxidoreductase activity Relationships: is a type of oxidoreductase activity, acting on the CH-CH group of donors, NAD or NADP as acceptor [GO:0016628]